{
  "term_label": "I-SMAD binding",
  "gene_symbol": "SMAD7",
  "gene_name": "Mothers against decapentaplegic homolog 7",
  "term_id": "GO:0070411",
  "gene": "UniProtKB:O15105"
}